{
  "gene": "UniProtKB:Q6TFL4",
  "term_id": "GO:0005737",
  "gene_name": "Kelch-like protein 24",
  "gene_symbol": "KLHL24",
  "term_label": "cytoplasm"
}